regulation of artery morphogenesis [GO:1905651] (biological process) References: PMID:27389411 Sources: GOC:BHF, GOC:BHF_miRNA, GOC:TermGenie, GOC:rph, GO_REF:0000058 Also known as: regulation of arterial morphogenesis, regulation of arteriogenesis Subtypes: GO:1903847, regulation of ductus arteriosus closure [GO:1904335], GO:1905652, positive regulation of artery morphogenesis [GO:1905653] Relationships: is a type of GO:0022603; regulates GO:0048844 Definition: Any process that modulates the frequency, rate or extent of artery morphogenesis.